 [rdf-schema#comment]